{
  "gene": "UniProtKB:Q9Y6R6",
  "gene_name": "Zinc finger protein 780B",
  "term_id": "GO:0006357",
  "term_label": "regulation of transcription by RNA polymerase II",
  "gene_symbol": "ZNF780B"
}